CD4-positive, alpha-beta T cell lineage commitment [GO:0043373] (biological process) Sources: ISBN:0781735149 Relationships: is a type of alpha-beta T cell lineage commitment [GO:0002363]; is a type of GO:0043369; BFO_0000050 CD4-positive, alpha-beta T cell differentiation [GO:0043367] Also known as: CD4-positive, alpha-beta T lymphocyte lineage commitment, CD4-positive, alpha-beta T-cell lineage commitment, CD4-positive, alpha-beta T-lymphocyte lineage commitment Subtypes: T-helper cell lineage commitment [GO:0002295], GO:0002362 Definition: The process in which an immature T cell becomes committed to becoming a CD4-positive, alpha-beta T cell.